{
  "gene_symbol": "SLC25A23",
  "term_id": "UNKNOWN:0003",
  "gene": "UniProtKB:Q9BV35",
  "gene_name": "Mitochondrial adenyl nucleotide antiporter SLC25A23",
  "term_label": "Unknown cellular component"
}